{
  "gene_name": "Nitric oxide synthase, inducible",
  "gene_symbol": "NOS2",
  "gene": "UniProtKB:P35228",
  "term_label": "nitric-oxide synthase activity",
  "term_id": "GO:0004517"
}